{
  "term_id": "GO:0000785",
  "gene": "UniProtKB:Q9NQB0",
  "term_label": "chromatin",
  "gene_name": "Transcription factor 7-like 2",
  "gene_symbol": "TCF7L2"
}